{
  "gene_name": "cAMP-regulated phosphoprotein 21",
  "gene": "UniProtKB:Q9UBL0",
  "term_label": "cytoplasm",
  "gene_symbol": "ARPP21",
  "term_id": "GO:0005737"
}